{
  "term_id": "GO:0072686",
  "gene": "UniProtKB:Q9BXS6",
  "term_label": "mitotic spindle",
  "gene_name": "Nucleolar and spindle-associated protein 1",
  "gene_symbol": "NUSAP1"
}